regulation of adenylate cyclase-inhibiting opioid receptor signaling pathway [GO:1900729] (BP) References: PMID:17157995 Sources: GOC:TermGenie, GOC:sjw Relationships: is_a regulation of opioid receptor signaling pathway [GO:2000474]; regulates GO:0031635 Subtypes: negative regulation of adenylate cyclase-inhibiting opioid receptor signaling pathway [GO:1900730], positive regulation of adenylate cyclase-inhibiting opioid receptor signaling pathway [GO:1900731] Also known as: regulation of inhibition of adenylate cyclase activity by opioid receptor, regulation of inhibition of adenylate cyclase activity by opioid receptor signaling pathway, regulation of inhibition of adenylate cyclase activity by opioid receptor signalling pathway, regulation of opioid receptor-mediated adenylate cyclase inhibition Definition: Any process that modulates the frequency, rate or extent of adenylate cyclase-inhibiting opioid receptor signaling pathway.